{
  "gene_name": "Ectonucleoside triphosphate diphosphohydrolase 7",
  "term_id": "GO:0046036",
  "gene_symbol": "ENTPD7",
  "term_label": "CTP metabolic process",
  "gene": "UniProtKB:Q9NQZ7"
}